{
  "gene_symbol": "MYL6B",
  "gene_name": "Myosin light chain 6B",
  "gene": "UniProtKB:P14649",
  "term_id": "GO:0000146",
  "term_label": "microfilament motor activity"
}